{
  "term_id": "GO:0045893",
  "term_label": "positive regulation of DNA-templated transcription",
  "gene_symbol": "TP53INP1",
  "gene_name": "Tumor protein p53-inducible nuclear protein 1",
  "gene": "UniProtKB:Q96A56"
}